poly(hydroxyvalerate) biosynthetic process [GO:1902921] (biological process) References: PMID:21705209 Sources: GOC:TermGenie, GOC:mengo_curators, GO_REF:0000068 Also known as: poly(hydroxyvalerate) anabolism, poly(hydroxyvalerate) biosynthesis, poly(hydroxyvalerate) formation, poly(hydroxyvalerate) synthesis Subtypes: poly(5-hydroxyvalerate) biosynthetic process [GO:1902919], poly(3-hydroxyvalerate) biosynthetic process [GO:1902923] Definition: The chemical reactions and pathways resulting in the formation of poly(hydroxyvalerate). Relationships: is_a poly(hydroxyalkanoate) biosynthetic process [GO:1901441]